{
  "gene_name": "Endosome_lysosome-associated apoptosis and autophagy regulator 1",
  "gene_symbol": "ELAPOR1",
  "term_id": "GO:0000045",
  "term_label": "autophagosome assembly",
  "gene": "UniProtKB:Q6UXG2"
}